{
  "gene": "UniProtKB:Q8N413",
  "term_id": "GO:0022857",
  "gene_name": "Solute carrier family 25 member 45",
  "term_label": "transmembrane transporter activity",
  "gene_symbol": "SLC25A45"
}